{
  "term_id": "GO:0007051",
  "gene": "UniProtKB:Q2M2Z5",
  "gene_name": "Centrosomal protein kizuna",
  "gene_symbol": "KIZ",
  "term_label": "spindle organization"
}